{
  "term_id": "UNKNOWN:0001",
  "gene": "UniProtKB:Q7L4P6",
  "gene_symbol": "BEND5",
  "gene_name": "BEN domain-containing protein 5",
  "term_label": "Unknown molecular function"
}